glyoxysome [GO:0009514] (cellular component) Definition: A specialized form of peroxisome that contains the enzymes of the glyoxylate pathway. The glyoxysome is found in some plant cells, notably the cells of germinating seeds. Relationships: is a type of peroxisome [GO:0005777] Sources: GOC:dhl, ISBN:0140514031